beta-glucanase activity [GO:0052736] (molecular function) Relationships: is a type of hydrolase activity, hydrolyzing O-glycosyl compounds [GO:0004553] Definition: Catalysis of the hydrolysis of linkages in beta-D-glucans; beta-glucans are polysaccharides of D-glucose monomers linked by beta-glycosidic bonds. Also known as: beta-D-glucanase activity Sources: Wikipedia:Beta-glucan Subtypes: GO:0033946, GO:0033950, endo-1,3(4)-beta-glucanase activity [GO:0052861]